{
  "gene": "UniProtKB:Q15738",
  "gene_name": "Sterol-4-alpha-carboxylate 3-dehydrogenase, decarboxylating",
  "term_id": "GO:0005783",
  "gene_symbol": "NSDHL",
  "term_label": "endoplasmic reticulum"
}